negative regulation of focal adhesion assembly [GO:0051895] (biological process) Definition: Any process that stops, prevents, or reduces the frequency, rate or extent of focal adhesion assembly, the establishment and maturation of focal adhesions. Also known as: down regulation of focal adhesion formation, down-regulation of focal adhesion formation, downregulation of focal adhesion formation, inhibition of focal adhesion formation Sources: GOC:ai Relationships: is a type of negative regulation of cell-matrix adhesion [GO:0001953]; is a type of regulation of focal adhesion assembly [GO:0051893]; is a type of negative regulation of cell-substrate junction organization [GO:0150118]; is a type of negative regulation of cell junction assembly [GO:1901889]; negatively regulates GO:0048041